{
  "term_id": "GO:0016558",
  "gene_symbol": "PEX10",
  "gene_name": "Peroxisome biogenesis factor 10",
  "gene": "UniProtKB:O60683",
  "term_label": "protein import into peroxisome matrix"
}